{
  "gene_symbol": "SLC22A15",
  "term_id": "UNKNOWN:0001",
  "gene": "UniProtKB:Q8IZD6",
  "gene_name": "Solute carrier family 22 member 15",
  "term_label": "Unknown molecular function"
}